regulation of silent mating-type cassette heterochromatin formation [GO:0090054] (biological process) Sources: GOC:dph, GOC:tb Definition: Any process that modulates the frequency, rate, or extent of heterochromatin formation at silent mating-type cassette. Relationships: is a type of regulation of heterochromatin formation [GO:0031445]; regulates silent mating-type cassette heterochromatin formation [GO:0030466] Subtypes: negative regulation of silent mating-type cassette heterochromatin formation [GO:0061186], GO:0090055 Also known as: regulation of chromatin silencing at silent mating-type cassette, regulation of silent mating-type cassette heterochromatin assembly